negative regulation of R7 cell fate commitment [GO:0106398] (biological process) References: PMID:22878552 Sources: GOC:ha Relationships: is a type of negative regulation of cell fate commitment [GO:0010454]; is a type of regulation of R7 cell fate commitment [GO:0106396]; negatively regulates R7 cell fate commitment [GO:0007465] Definition: Any process that stops, prevents or reduces the frequency, rate or extent of R7 cell fate commitment.